{
  "gene": "UniProtKB:P35218",
  "term_label": "cytoplasm",
  "gene_symbol": "CA5A",
  "gene_name": "Carbonic anhydrase 5A, mitochondrial",
  "term_id": "GO:0005737"
}